{
  "term_id": "GO:0043001",
  "gene": "UniProtKB:Q8N2H4",
  "term_label": "Golgi to plasma membrane protein transport",
  "gene_symbol": "SYS1",
  "gene_name": "Protein SYS1 homolog"
}